{
  "gene": "UniProtKB:Q7Z5W3",
  "term_label": "negative regulation of pre-miRNA processing",
  "term_id": "GO:2000632",
  "gene_name": "RNA 5'-monophosphate methyltransferase",
  "gene_symbol": "BCDIN3D"
}